{
  "gene_name": "Solute carrier family 15 member 3",
  "term_label": "lysosomal membrane",
  "gene_symbol": "SLC15A3",
  "term_id": "GO:0005765",
  "gene": "UniProtKB:Q8IY34"
}